{
  "gene_name": "Semaphorin-5A",
  "gene": "UniProtKB:Q13591",
  "term_label": "chemorepellent activity",
  "term_id": "GO:0045499",
  "gene_symbol": "SEMA5A"
}